{
  "gene_name": "Interleukin-1 alpha",
  "gene": "UniProtKB:P01583",
  "term_label": "positive regulation of canonical NF-kappaB signal transduction",
  "term_id": "GO:0043123",
  "gene_symbol": "IL1A"
}